{
  "gene": "UniProtKB:P62826",
  "gene_name": "GTP-binding nuclear protein Ran",
  "term_id": "GO:0006606",
  "gene_symbol": "RAN",
  "term_label": "protein import into nucleus"
}